CLOCK-BMAL transcription complex [GO:1990513] (cellular component) References: PMID:23229515 Sources: GOC:bhm Note: An example of this is CLOCK in human (O15516) in PMID:23229515 (inferred from physical interaction). Also known as: CLOCK/BMAL complex Relationships: is a type of RNA polymerase II transcription regulator complex [GO:0090575] Definition: Transcription factor complex which interacts with E-box regulatory elements in target genes, including Period (Per1, Per2, Per3) and Cryptochrome (Cry1, Cry2), to activate their transcription during the daytime. The CRY-PER complexes inhibit CLOCK-BMAL1-driven transcription in a negative feedback loop to generate circadian rhythms.